positive regulation of convergent extension involved in axis elongation [GO:1901234] (BP) Relationships: is a type of positive regulation of developmental growth [GO:0048639]; is_a regulation of convergent extension involved in axis elongation [GO:1901232]; is a type of positive regulation of morphogenesis of an epithelium [GO:1905332]; RO_0002213 convergent extension involved in axis elongation [GO:0060028] Sources: GOC:BHF, GOC:TermGenie Subtypes: positive regulation of convergent extension involved in somitogenesis [GO:1904129] Also known as: up regulation of convergent extension involved in axis elongation, up-regulation of convergent extension involved in axis elongation, upregulation of convergent extension involved in axis elongation, activation of convergent extension involved in axis elongation Definition: Any process that activates or increases the frequency, rate or extent of convergent extension involved in axis elongation.